7-methylguanosine RNA capping [GO:0009452] (biological process) References: PMID:9266685 Sources: GOC:vw Subtypes: GO:0006370 Relationships: is a type of RNA capping [GO:0036260] Definition: The sequence of enzymatic reactions by which the RNA 5' cap structure, an inverted 7-methylguanosine linked via a 5'-5' triphosphate bridge (m7G(5')ppp(5')X) to the first transcribed residue, is added to a nascent transcript. Additional methylation can occur on the ribose sugars of the first and second nucleotides adjacent to the m7G nRNA cap. These methylations are often referred to as N6,2'-O-dimethyladenosine (m6,2A) and N6,2'-O-dimethylguanosine (m6,2G), respectively. Also known as: RNA capping, m(7)G RNA capping